{
  "gene": "UniProtKB:P68036",
  "gene_symbol": "UBE2L3",
  "term_label": "nucleus",
  "gene_name": "Ubiquitin-conjugating enzyme E2 L3",
  "term_id": "GO:0005634"
}